{
  "gene": "UniProtKB:A0A075B714",
  "gene_symbol": "TRAJ7",
  "gene_name": "T cell receptor alpha joining 7 (Fragment)",
  "term_label": "Unknown cellular component",
  "term_id": "UNKNOWN:0003"
}